{
  "gene": "UniProtKB:Q5TB80",
  "gene_name": "Centrosomal protein of 162 kDa",
  "gene_symbol": "CEP162",
  "term_label": "nucleoplasm",
  "term_id": "GO:0005654"
}